{
  "term_label": "intraciliary retrograde transport",
  "gene_symbol": "IFT140",
  "gene": "UniProtKB:Q96RY7",
  "term_id": "GO:0035721",
  "gene_name": "Intraflagellar transport protein 140 homolog"
}